{
  "gene_name": "Early growth response protein 3",
  "term_id": "GO:0000978",
  "gene": "UniProtKB:Q06889",
  "gene_symbol": "EGR3",
  "term_label": "RNA polymerase II cis-regulatory region sequence-specific DNA binding"
}